{
  "gene_name": "T cell receptor delta variable 2",
  "term_id": "UNKNOWN:0002",
  "gene_symbol": "TRDV2",
  "gene": "UniProtKB:A0JD36",
  "term_label": "Unknown biological process"
}